{
  "gene_name": "Testis-expressed protein 26",
  "gene_symbol": "TEX26",
  "term_label": "Unknown biological process",
  "gene": "UniProtKB:Q8N6G2",
  "term_id": "UNKNOWN:0002"
}